{
  "gene_name": "Probable ATP-dependent RNA helicase DDX53",
  "gene_symbol": "DDX53",
  "gene": "UniProtKB:Q86TM3",
  "term_label": "Unknown biological process",
  "term_id": "UNKNOWN:0002"
}